{
  "term_id": "GO:0006936",
  "gene": "UniProtKB:Q9Y623",
  "gene_name": "Myosin-4",
  "gene_symbol": "MYH4",
  "term_label": "muscle contraction"
}